defense response to fungus [GO:0050832] (biological process) Relationships: is a type of defense response [GO:0006952]; is a type of response to fungus [GO:0009620] Subtypes: antifungal humoral response [GO:0019732], antifungal innate immune response [GO:0061760] Sources: GOC:ai Definition: Reactions triggered in response to the presence of a fungus that act to protect the cell or organism. Also known as: defence response to fungi, defence response to fungus, defense response to fungi, defense response to fungus, incompatible interaction, resistance response to pathogenic fungi, resistance response to pathogenic fungus, response to parasitic fungi, response to parasitic fungus Regulation: regulated by regulation of defense response to fungus [GO:1900150]